{
  "term_label": "canonical NF-kappaB signal transduction",
  "gene": "UniProtKB:Q04864",
  "gene_symbol": "REL",
  "term_id": "GO:0007249",
  "gene_name": "Proto-oncogene c-Rel"
}